regulation of type B pancreatic cell apoptotic process [GO:2000674] (BP) Also known as: regulation of pancreatic B cell apoptosis, regulation of pancreatic beta cell apoptosis, regulation of type B pancreatic cell apoptosis Relationships: is a type of regulation of epithelial cell apoptotic process [GO:1904035]; regulates type B pancreatic cell apoptotic process [GO:0097050] Sources: GOC:mtg_apoptosis, GOC:obol Definition: Any process that modulates the frequency, rate or extent of type B pancreatic cell apoptotic process. Subtypes: GO:2000675, GO:2000676